{
  "gene_name": "Olfactory receptor 8D4",
  "term_label": "olfactory receptor activity",
  "gene": "UniProtKB:Q8NGM9",
  "gene_symbol": "OR8D4",
  "term_id": "GO:0004984"
}